RNA polymerase core enzyme binding [GO:0043175] (molecular function) Sources: GOC:jl, GOC:txnOH Definition: Binding to an RNA polymerase core enzyme, containing a specific subunit composition defined as the core enzyme. Subtypes: GO:0000993, GO:0000994, bacterial-type RNA polymerase core enzyme binding [GO:0001000], RNA polymerase I core binding [GO:0001042], RNA polymerase IV core binding [GO:0001048], GO:0001049 Relationships: is a type of RNA polymerase binding [GO:0070063]